{
  "gene_symbol": "IER5",
  "gene": "UniProtKB:Q5VY09",
  "gene_name": "Immediate early response gene 5 protein",
  "term_id": "UNKNOWN:0002",
  "term_label": "Unknown biological process"
}